axon collateral [GO:0044303] (cellular component) Relationships: is a type of GO:0110165; is part of axon [GO:0030424] Definition: Any of the smaller branches of an axon that emanate from the main axon cylinder. Sources: NIF_Subcellular:sao1470140754 Subtypes: recurrent axon collateral [GO:1990020], Schaffer axon collateral [GO:1990021]